cellular response to nitrogen dioxide [GO:0035714] (biological process) Sources: GOC:BHF Also known as: cellular response to NO2 Definition: Any process that results in a change in state or activity of a cell (in terms of movement, secretion, enzyme production, gene expression, etc.) as a result of a nitrogen dioxide (NO2) stimulus. Relationships: is a type of response to nitrogen dioxide [GO:0035713]; is a type of cellular response to nitrogen compound [GO:1901699]; is a type of cellular response to oxygen-containing compound [GO:1901701]